stachyose biosynthetic process [GO:0033532] (biological process) Also known as: stachyose anabolism, stachyose biosynthesis, stachyose formation, stachyose synthesis Sources: GOC:mah Relationships: is a type of raffinose family oligosaccharide biosynthetic process [GO:0010325]; is a type of stachyose metabolic process [GO:0033531] Definition: The chemical reactions and pathways resulting in the formation of stachyose, the tetrasaccharide beta-D-fructofuranosyl alpha-D-galactopyranosyl-(1->6)-alpha-D-galactopyranosyl-(1->6)-alpha-D-glucopyranoside.